cell-cell adhesion involved in ameboidal cell migration [GO:0003367] (biological process) Relationships: is a type of cell-cell adhesion [GO:0098609]; is part of establishment of cell polarity involved in ameboidal cell migration [GO:0003365] Definition: The attachment of one ameboid cell to another that contributes to the establishment of cell polarity that is part of the directed movement of one of the cells. Subtypes: cell-cell adhesion involved in mesendodermal cell migration [GO:0003370] Sources: GOC:ascb_2009, GOC:dph, GOC:tb